{
  "term_id": "GO:0006357",
  "gene": "UniProtKB:O43313",
  "term_label": "regulation of transcription by RNA polymerase II",
  "gene_name": "ATM interactor",
  "gene_symbol": "ATMIN"
}